{
  "term_label": "site of double-strand break",
  "gene": "UniProtKB:Q8NCN4",
  "gene_name": "E3 ubiquitin-protein ligase RNF169",
  "term_id": "GO:0035861",
  "gene_symbol": "RNF169"
}